formation of syncytium involving giant cell for nutrient acquisition [GO:0052096] (biological process) Also known as: formation by organism of syncytium involving giant cell for nutrient acquisition from host, formation by symbiont of syncytium involving giant cell for nutrient acquisition from host Relationships: is a type of formation of specialized structure for nutrient acquisition [GO:0052093] Definition: The assembly of a syncytium, a multi-nucleate and physiologically active aggregation of fused root cells induced by a symbiotic nematode in a plant host. The syncytium exclusively provides the nematode with nourishment during its sedentary life, for the purpose of obtaining nutrients from its host organism. The host is defined as the larger of the organisms involved in a symbiotic interaction. Sources: GOC:pamgo_curators